{
  "term_id": "GO:0045143",
  "gene_name": "Securin",
  "gene_symbol": "PTTG1",
  "gene": "UniProtKB:O95997",
  "term_label": "homologous chromosome segregation"
}